aortic valve formation [GO:0003189] (biological process) Sources: GOC:mtg_heart Definition: The developmental process pertaining to the initial formation of the aortic valve from unspecified parts. This process begins with the specific processes that contribute to the appearance of the discrete structure and ends when the structural rudiment is recognizable. Relationships: is a type of heart valve formation [GO:0003188]; is part of aortic valve morphogenesis [GO:0003180]